{
  "term_id": "GO:0036126",
  "term_label": "sperm flagellum",
  "gene": "UniProtKB:Q9H112",
  "gene_symbol": "CST11",
  "gene_name": "Cystatin-11"
}